{
  "gene_symbol": "MYL9",
  "gene": "UniProtKB:P24844",
  "term_label": "cytoplasm",
  "gene_name": "Myosin regulatory light polypeptide 9",
  "term_id": "GO:0005737"
}